{
  "term_id": "GO:0005774",
  "gene_symbol": "SLC36A3",
  "gene": "UniProtKB:Q495N2",
  "gene_name": "Proton-coupled amino acid transporter 3",
  "term_label": "vacuolar membrane"
}